{
  "term_id": "GO:0005854",
  "gene_symbol": "BTF3",
  "gene_name": "Transcription factor BTF3",
  "gene": "UniProtKB:P20290",
  "term_label": "nascent polypeptide-associated complex"
}